{
  "gene_name": "Histone H2B type 1-J",
  "gene": "UniProtKB:P06899",
  "gene_symbol": "H2BC11",
  "term_id": "GO:0000786",
  "term_label": "nucleosome"
}